{
  "gene": "UniProtKB:Q8N878",
  "term_label": "plasma membrane",
  "gene_name": "FERM domain-containing protein 1",
  "gene_symbol": "FRMD1",
  "term_id": "GO:0005886"
}